{
  "gene_symbol": "C8A",
  "gene": "UniProtKB:P07357",
  "term_id": "GO:0006956",
  "gene_name": "Complement component C8 alpha chain",
  "term_label": "complement activation"
}